indeterminate inflorescence morphogenesis [GO:0048283] (BP) Sources: GOC:jid Relationships: is a type of GO:0048281 Definition: The process in which the anatomical structures of determinate inflorescences are generated and organized. A determinate inflorescence is one that can produce an undefined number of floral meristems.